{
  "gene_symbol": "PDE3A",
  "term_label": "3',5'-cyclic-AMP phosphodiesterase activity",
  "term_id": "GO:0004115",
  "gene": "UniProtKB:Q14432",
  "gene_name": "cGMP-inhibited 3',5'-cyclic phosphodiesterase 3A"
}